activation of protein kinase activity [GO:0032147] (biological process) Definition: Any process that initiates the activity of an inactive protein kinase. Sources: GOC:mah Also known as: protein kinase activation Relationships: is a type of positive regulation of protein kinase activity [GO:0045860] Subtypes: activation of transmembrane receptor protein tyrosine kinase activity [GO:0007171], GO:0007250, activation of protein kinase B activity [GO:0032148], activation of protein kinase A activity [GO:0034199], activation of Janus kinase activity [GO:0042976], activation of protein kinase C activity [GO:1990051]